{
  "term_id": "UNKNOWN:0003",
  "gene_symbol": "KLHDC7A",
  "gene": "UniProtKB:Q5VTJ3",
  "term_label": "Unknown cellular component",
  "gene_name": "Kelch domain-containing protein 7A"
}